{
  "gene_symbol": "EMD",
  "term_id": "GO:0048487",
  "gene": "UniProtKB:P50402",
  "gene_name": "Emerin",
  "term_label": "beta-tubulin binding"
}